{
  "term_label": "Unknown cellular component",
  "term_id": "UNKNOWN:0003",
  "gene_symbol": "PGA4",
  "gene_name": "Pepsin A-4",
  "gene": "UniProtKB:P0DJD7"
}